{
  "term_label": "synaptic vesicle docking",
  "gene_symbol": "RIMS2",
  "term_id": "GO:0016081",
  "gene": "UniProtKB:Q9UQ26",
  "gene_name": "Regulating synaptic membrane exocytosis protein 2"
}